plant-type cell wall cellulose metabolic process [GO:0052541] (biological process) Definition: The chemical reactions and pathways involving cellulose, a linear beta1-4 glucan of molecular mass 50-400 kDa with the pyranose units in the -4C1 conformation, as part of the organization and biogenesis of the cell wall. Relationships: is a type of cellulose metabolic process [GO:0030243]; is a type of cell wall beta-glucan metabolic process [GO:0034406]; is part of plant-type cell wall organization [GO:0009664] Subtypes: plant-type cell wall cellulose catabolic process [GO:0044348], plant-type cell wall cellulose biosynthetic process [GO:0052324] Also known as: cell wall cellulose metabolism, cellulose and pectin-containing cell wall cellulose metabolic process Sources: GOC:mah, ISBN:0198506732